{
  "gene_name": "E3 ubiquitin-protein ligase RNF125",
  "term_label": "VCP-NPL4-UFD1 AAA ATPase complex",
  "term_id": "GO:0034098",
  "gene_symbol": "RNF125",
  "gene": "UniProtKB:Q96EQ8"
}